23S rRNA (adenine(2085)-N(6))-dimethyltransferase activity [GO:0052910] (molecular function) Definition: Catalysis of the reaction: 2 S-adenosyl-L-methionine + adenine(2085) in 23S rRNA = 2 S-adenosyl-L-homocysteine + N(6)-dimethyladenine(2085) in 23S rRNA. Sources: RHEA:42784 Also known as: ermC 23S rRNA methyltransferase activity, rRNA methyltransferase ermC' activity, rRNA:m(6)A methyltransferase ermC' activity Relationships: is_a rRNA (adenine-N6-)-methyltransferase activity [GO:0008988]